{
  "gene_symbol": "NBPF12",
  "term_id": "UNKNOWN:0001",
  "gene_name": "Neuroblastoma breakpoint family member 12",
  "gene": "UniProtKB:Q5TAG4",
  "term_label": "Unknown molecular function"
}